{
  "term_label": "intracellular calcium ion homeostasis",
  "gene_symbol": "EDN1",
  "term_id": "GO:0006874",
  "gene": "UniProtKB:P05305",
  "gene_name": "Endothelin-1"
}